{
  "term_label": "exopolyphosphatase activity",
  "gene_name": "Exopolyphosphatase PRUNE1",
  "gene": "UniProtKB:Q86TP1",
  "gene_symbol": "PRUNE1",
  "term_id": "GO:0004309"
}